{
  "gene": "UniProtKB:Q56P03",
  "term_id": "UNKNOWN:0002",
  "gene_name": "E2F-associated phosphoprotein",
  "gene_symbol": "EAPP",
  "term_label": "Unknown biological process"
}